gerontoplast stroma [GO:1905506] (CC) References: PMID:11212360 Sources: GOC:TermGenie, GOC:mag, GO_REF:0000064 Relationships: is a type of plastid stroma [GO:0009532]; is part of gerontoplast [GO:0034400] Definition: Any plastid stroma that is part of a gerontoplast.